response to pyrethroid [GO:0046684] (biological process) Relationships: is a type of response to insecticide [GO:0017085] Definition: Any process that results in a change in state or activity of a cell or an organism (in terms of movement, secretion, enzyme production, gene expression, etc.) as a result of a pyrethroid stimulus. Pyrethroids are a group of growth regulators, analogous to insect juvenile hormones, that interfere with the development of insect larvae and are used in the control of insects that are harmful in the adult stage. Sources: ISBN:0721662544 Also known as: pyrethroid resistance, pyrethroid susceptibility/resistance